{
  "gene_name": "Integral membrane protein 2C",
  "term_label": "plasma membrane",
  "term_id": "GO:0005886",
  "gene_symbol": "ITM2C",
  "gene": "UniProtKB:Q9NQX7"
}